{
  "gene_symbol": "B3GALT2",
  "term_id": "GO:0006682",
  "term_label": "galactosylceramide biosynthetic process",
  "gene_name": "Beta-1,3-galactosyltransferase 2",
  "gene": "UniProtKB:O43825"
}